cardiac muscle hypertrophy in response to stress [GO:0014898] (biological process) Definition: The physiological enlargement or overgrowth of all or part of the heart muscle due to an increase in size (not length) of individual cardiac muscle fibers, without cell division, as a result of a disturbance in organismal or cellular homeostasis. Relationships: is a type of muscle hypertrophy in response to stress [GO:0003299]; is a type of cardiac muscle hypertrophy [GO:0003300]; is a type of cardiac muscle adaptation [GO:0014887] Regulation: regulated by GO:1903242; negatively regulated by negative regulation of cardiac muscle hypertrophy in response to stress [GO:1903243]; positively regulated by GO:1903244 Sources: GOC:BHF, GOC:mtg_cardiac_conduct_nov11, GOC:mtg_muscle